{
  "gene_name": "Galectin-9B",
  "term_id": "GO:0030246",
  "gene": "UniProtKB:Q3B8N2",
  "gene_symbol": "LGALS9B",
  "term_label": "carbohydrate binding"
}